{
  "gene_name": "Zinc finger protein 98",
  "term_label": "DNA-binding transcription factor activity, RNA polymerase II-specific",
  "term_id": "GO:0000981",
  "gene_symbol": "ZNF98",
  "gene": "UniProtKB:A6NK75"
}